host cell Golgi apparatus [GO:0044177] (cellular component) Relationships: is_a host cell cytoplasm part [GO:0033655] Definition: A compound membranous cytoplasmic organelle of eukaryotic host cells, consisting of flattened, ribosome-free vesicles arranged in a more or less regular stack. Sources: GOC:jl Also known as: host Golgi apparatus